{
  "term_id": "UNKNOWN:0002",
  "term_label": "Unknown biological process",
  "gene_symbol": "SCYL3",
  "gene_name": "Protein-associating with the carboxyl-terminal domain of ezrin",
  "gene": "UniProtKB:Q8IZE3"
}